{
  "gene_name": "Smoothelin-like protein 2",
  "gene": "UniProtKB:Q2TAL5",
  "gene_symbol": "SMTNL2",
  "term_id": "UNKNOWN:0001",
  "term_label": "Unknown molecular function"
}